{
  "gene_name": "Non-receptor tyrosine-protein kinase TYK2",
  "term_id": "GO:0060397",
  "gene_symbol": "TYK2",
  "term_label": "growth hormone receptor signaling pathway via JAK-STAT",
  "gene": "UniProtKB:P29597"
}